{
  "gene_symbol": "SMARCD3",
  "gene_name": "SWI_SNF-related matrix-associated actin-dependent regulator of chromatin subfamily D member 3",
  "gene": "UniProtKB:Q6STE5",
  "term_label": "nucleus",
  "term_id": "GO:0005634"
}